{
  "term_label": "L-malate dehydrogenase (NAD+) activity",
  "gene_symbol": "MDH1",
  "gene": "UniProtKB:P40925",
  "gene_name": "Malate dehydrogenase, cytoplasmic",
  "term_id": "GO:0030060"
}